{
  "gene_name": "Ficolin-3",
  "term_id": "GO:0031012",
  "term_label": "extracellular matrix",
  "gene_symbol": "FCN3",
  "gene": "UniProtKB:O75636"
}